cranial nerve morphogenesis [GO:0021602] (biological process) Relationships: is a type of anatomical structure morphogenesis [GO:0009653]; is part of GO:0021545 Definition: The process in which the anatomical structure of the cranial nerves are generated and organized. The cranial nerves are composed of twelve pairs of nerves that emanate from the nervous tissue of the hindbrain. These nerves are sensory, motor, or mixed in nature, and provide the motor and general sensory innervation of the head, neck and viscera. They mediate vision, hearing, olfaction and taste and carry the parasympathetic innervation of the autonomic ganglia that control visceral functions. Subtypes: abducens nerve morphogenesis [GO:0021598], GO:0021607, facial nerve morphogenesis [GO:0021610], glossopharyngeal nerve morphogenesis [GO:0021615], hypoglossal nerve morphogenesis [GO:0021618], oculomotor nerve morphogenesis [GO:0021622], olfactory nerve morphogenesis [GO:0021627], optic nerve morphogenesis [GO:0021631], trigeminal nerve morphogenesis [GO:0021636], GO:0021639, vagus nerve morphogenesis [GO:0021644], vestibulocochlear nerve morphogenesis [GO:0021648] Sources: GOC:cls, GOC:dgh, GOC:dph, GOC:jid, GO_REF:0000021